{
  "gene": "UniProtKB:Q8NBT0",
  "term_id": "GO:0036064",
  "gene_name": "POC1 centriolar protein homolog A",
  "term_label": "ciliary basal body",
  "gene_symbol": "POC1A"
}